{
  "gene_symbol": "PGLYRP4",
  "gene_name": "Peptidoglycan recognition protein 4",
  "term_label": "N-acetylmuramoyl-L-alanine amidase activity",
  "gene": "UniProtKB:Q96LB8",
  "term_id": "GO:0008745"
}